{
  "gene": "UniProtKB:Q9NX57",
  "gene_name": "Ras-related protein Rab-20",
  "gene_symbol": "RAB20",
  "term_label": "endomembrane system",
  "term_id": "GO:0012505"
}